{
  "gene": "UniProtKB:A0A0C4DH62",
  "gene_symbol": "IGHJ1",
  "term_id": "UNKNOWN:0001",
  "term_label": "Unknown molecular function",
  "gene_name": "Immunoglobulin heavy joining 1"
}